{
  "gene_symbol": "ARL11",
  "gene_name": "ADP-ribosylation factor-like protein 11",
  "gene": "UniProtKB:Q969Q4",
  "term_label": "plasma membrane",
  "term_id": "GO:0005886"
}